{
  "term_label": "Unknown cellular component",
  "gene_symbol": "SEC22B",
  "term_id": "UNKNOWN:0003",
  "gene_name": "Vesicle-trafficking protein SEC22b",
  "gene": "UniProtKB:O75396"
}